{
  "gene": "UniProtKB:Q5T8D3",
  "term_id": "GO:0006631",
  "term_label": "fatty acid metabolic process",
  "gene_name": "Acyl-CoA-binding domain-containing protein 5",
  "gene_symbol": "ACBD5"
}